{
  "gene_symbol": "PRLH",
  "gene_name": "Prolactin-releasing peptide",
  "term_label": "neuropeptide hormone activity",
  "gene": "UniProtKB:P81277",
  "term_id": "GO:0005184"
}